{
  "term_label": "apoptotic process",
  "gene_name": "E3 ubiquitin-protein ligase TRAF7",
  "gene": "UniProtKB:Q6Q0C0",
  "term_id": "GO:0006915",
  "gene_symbol": "TRAF7"
}